{
  "term_label": "establishment or maintenance of cell polarity",
  "gene_name": "Rho-related BTB domain-containing protein 1",
  "gene_symbol": "RHOBTB1",
  "gene": "UniProtKB:O94844",
  "term_id": "GO:0007163"
}